{
  "term_label": "1-alkyl-2-acetylglycerophosphocholine esterase activity",
  "term_id": "GO:0003847",
  "gene_name": "Platelet-activating factor acetylhydrolase 2, cytoplasmic",
  "gene_symbol": "PAFAH2",
  "gene": "UniProtKB:Q99487"
}